{
  "gene_symbol": "TMEM259",
  "term_label": "endoplasmic reticulum",
  "term_id": "GO:0005783",
  "gene_name": "Membralin",
  "gene": "UniProtKB:Q4ZIN3"
}